{
  "term_label": "Unknown cellular component",
  "gene": "UniProtKB:Q9P1U1",
  "gene_symbol": "ACTR3B",
  "gene_name": "Actin-related protein 3B",
  "term_id": "UNKNOWN:0003"
}